{
  "gene_name": "Ephrin-B1",
  "term_id": "GO:0007411",
  "gene": "UniProtKB:P98172",
  "gene_symbol": "EFNB1",
  "term_label": "axon guidance"
}